{
  "term_label": "oxidative phosphorylation uncoupler activity",
  "gene_name": "Dicarboxylate carrier SLC25A8",
  "gene": "UniProtKB:P55851",
  "gene_symbol": "UCP2",
  "term_id": "GO:0017077"
}